{
  "gene": "UniProtKB:P55083",
  "gene_name": "Microfibril-associated glycoprotein 4",
  "term_label": "elastic fiber assembly",
  "gene_symbol": "MFAP4",
  "term_id": "GO:0048251"
}